clathrin binding [GO:0030276] (molecular function) Sources: GOC:jl, GOC:mah, ISBN:0198506732 Relationships: is a type of protein binding [GO:0005515] Subtypes: GO:0032050, clathrin light chain binding [GO:0032051] Definition: Binding to a clathrin heavy or light chain, the main components of the coat of coated vesicles and coated pits, and which also occurs in synaptic vesicles.